regulation of nitric-oxide synthase activity [GO:0050999] (biological process) Also known as: NOS regulator, nitric-oxide synthase regulator, regulation of NOS activity Sources: GOC:ai Relationships: is a type of regulation of oxidoreductase activity [GO:0051341]; regulates GO:0004517 Subtypes: positive regulation of nitric-oxide synthase activity [GO:0051000], GO:0051001 Definition: Any process that modulates the activity of the enzyme nitric-oxide synthase.